{
  "gene": "UniProtKB:P26447",
  "gene_name": "Protein S100-A4",
  "term_label": "positive regulation of canonical NF-kappaB signal transduction",
  "gene_symbol": "S100A4",
  "term_id": "GO:0043123"
}